{
  "gene": "UniProtKB:A0A0G2JNJ9",
  "term_id": "UNKNOWN:0001",
  "gene_name": "Uncharacterized protein",
  "gene_symbol": "A0A0G2JNJ9",
  "term_label": "Unknown molecular function"
}